{
  "gene_name": "Unconventional myosin-Ig",
  "term_label": "microfilament motor activity",
  "gene_symbol": "MYO1G",
  "term_id": "GO:0000146",
  "gene": "UniProtKB:B0I1T2"
}